{
  "term_label": "positive regulation of canonical Wnt signaling pathway",
  "gene_name": "Proto-oncogene FRAT1",
  "gene": "UniProtKB:Q92837",
  "gene_symbol": "FRAT1",
  "term_id": "GO:0090263"
}